regulation of attachment of spindle microtubules to kinetochore [GO:0051988] (biological process) Sources: GOC:ai Subtypes: GO:0051986, positive regulation of attachment of spindle microtubules to kinetochore [GO:0051987], GO:1902423, regulation of spindle attachment to meiosis I kinetochore [GO:1904967] Relationships: is_a regulation of cell cycle process [GO:0010564]; regulates GO:0008608 Also known as: regulation of kinetochore-microtubule attachment Definition: Any process that modulates the frequency, rate or extent of the attachment of spindle microtubules to the kinetochore.